detection of external biotic stimulus [GO:0098581] (biological process) Subtypes: detection of molecule of bacterial origin [GO:0032490], GO:0032491, detection of molecule of oomycetes origin [GO:0032492], GO:0098543 Relationships: is a type of detection of biotic stimulus [GO:0009595]; is a type of GO:0043207 Definition: The series of events in which an external biotic stimulus is detected and converted into a molecular signal. An external biotic stimulus is defined as one caused or produced by a living organism other than the one being stimulated. Sources: GOC:dos Also known as: detection of exogenous biotic stimulus